{
  "gene_symbol": "OR13C7",
  "gene": "UniProtKB:P0DN81",
  "gene_name": "Olfactory receptor 13C7",
  "term_label": "detection of chemical stimulus involved in sensory perception of smell",
  "term_id": "GO:0050911"
}